regulation of cellular response to transforming growth factor beta stimulus [GO:1903844] (biological process) Definition: Any process that modulates the frequency, rate or extent of cellular response to transforming growth factor beta stimulus. Also known as: regulation of cellular response to TGF-beta stimulus, regulation of cellular response to TGFbeta stimulus Relationships: is a type of regulation of cellular response to growth factor stimulus [GO:0090287]; regulates GO:0071560 Subtypes: regulation of transforming growth factor beta receptor signaling pathway [GO:0017015], negative regulation of cellular response to transforming growth factor beta stimulus [GO:1903845], positive regulation of cellular response to transforming growth factor beta stimulus [GO:1903846] References: PMID:22269326 Sources: GOC:BHF, GOC:BHF_miRNA, GOC:TermGenie, GOC:rph, GO_REF:0000058